deoxyribonucleotide catabolic process [GO:0009264] (biological process) Also known as: deoxyribonucleotide breakdown, deoxyribonucleotide catabolism, deoxyribonucleotide degradation Sources: GOC:go_curators, ISBN:0198506732 Subtypes: purine deoxyribonucleotide catabolic process [GO:0009155], pyrimidine deoxyribonucleotide catabolic process [GO:0009223] Definition: The chemical reactions and pathways resulting in the breakdown of a deoxyribonucleotide, a compound consisting of deoxyribonucleoside (a base linked to a deoxyribose sugar) esterified with a phosphate group at either the 3' or 5'-hydroxyl group of the sugar. Relationships: is a type of nucleotide catabolic process [GO:0009166]; is a type of deoxyribonucleotide metabolic process [GO:0009262]; is a type of carbohydrate derivative catabolic process [GO:1901136]